positive regulation of endodeoxyribonuclease activity [GO:0032079] (biological process) Also known as: up regulation of endodeoxyribonuclease activity, up-regulation of endodeoxyribonuclease activity, upregulation of endodeoxyribonuclease activity, activation of endodeoxyribonuclease activity, stimulation of endodeoxyribonuclease activity, endodeoxyribonuclease activator Sources: GOC:mah Definition: Any process that activates or increases the frequency, rate or extent of endodeoxyribonuclease activity, the hydrolysis of ester linkages within deoxyribonucleic acid by creating internal breaks. Relationships: is a type of GO:0032071; is a type of positive regulation of deoxyribonuclease activity [GO:0032077]; positively regulates DNA endonuclease activity [GO:0004520]